{
  "gene_symbol": "IGKV1-8",
  "term_label": "immune response",
  "term_id": "GO:0006955",
  "gene_name": "Immunoglobulin kappa variable 1-8",
  "gene": "UniProtKB:A0A0C4DH67"
}